irritable aggressive behavior [GO:0002123] (biological process) Definition: Aggressive behavior induced by frustration and directed against an available target. Also known as: irritable aggression Relationships: is a type of aggressive behavior [GO:0002118] Sources: GOC:hjd